{
  "gene": "UniProtKB:Q8N6K4",
  "gene_name": "Putative uncharacterized protein MGC34800",
  "gene_symbol": "Q8N6K4",
  "term_id": "UNKNOWN:0002",
  "term_label": "Unknown biological process"
}